{
  "gene": "UniProtKB:Q96EK6",
  "gene_symbol": "GNPNAT1",
  "term_id": "GO:0004343",
  "gene_name": "Glucosamine 6-phosphate N-acetyltransferase",
  "term_label": "glucosamine 6-phosphate N-acetyltransferase activity"
}